{
  "gene_name": "Beta-3 adrenergic receptor",
  "term_id": "GO:0005886",
  "term_label": "plasma membrane",
  "gene_symbol": "ADRB3",
  "gene": "UniProtKB:P13945"
}